{
  "gene_symbol": "PDIK1L",
  "gene_name": "Serine_threonine-protein kinase PDIK1L",
  "term_label": "protein kinase activity",
  "gene": "UniProtKB:Q8N165",
  "term_id": "GO:0004672"
}